{
  "gene_symbol": "CARNS1",
  "gene": "UniProtKB:A5YM72",
  "term_label": "carnosine synthase activity",
  "term_id": "GO:0047730",
  "gene_name": "Carnosine synthase 1"
}